pigment granule transport [GO:0051904] (biological process) Definition: The directed movement of pigment granules into, out of or within a cell, or between cells, by means of some agent such as a transporter or pore. Subtypes: melanosome transport [GO:0032402] Also known as: pigment granule translocation Relationships: is a type of transport [GO:0006810]; is a type of pigment granule localization [GO:0051875]; is a type of establishment of pigment granule localization [GO:0051905] Sources: GOC:ai